interleukin-21 production [GO:0032625] (biological process) Sources: GOC:mah Also known as: IL-21 production, interleukin-21 biosynthetic process, interleukin-21 secretion Relationships: is a type of cytokine production [GO:0001816] Regulation: regulated by regulation of interleukin-21 production [GO:0032665]; negatively regulated by negative regulation of interleukin-21 production [GO:0032705]; positively regulated by positive regulation of interleukin-21 production [GO:0032745] Definition: The appearance of interleukin-21 due to biosynthesis or secretion following a cellular stimulus, resulting in an increase in its intracellular or extracellular levels.